cell proliferation in hindbrain [GO:0021534] (biological process) Sources: GOC:cls, GOC:dgh, GOC:dph, GOC:jid, GO_REF:0000021 Subtypes: GO:0021923, cell proliferation in external granule layer [GO:0021924] Relationships: is a type of neural precursor cell proliferation [GO:0061351]; is part of hindbrain development [GO:0030902] Definition: The multiplication or reproduction of cells, resulting in the expansion of a cell population in the hindbrain.